{
  "term_id": "GO:0005737",
  "term_label": "cytoplasm",
  "gene_name": "Signal transducer and activator of transcription 4",
  "gene_symbol": "STAT4",
  "gene": "UniProtKB:Q14765"
}